{
  "gene_symbol": "RIGI",
  "gene_name": "Antiviral innate immune response receptor RIG-I",
  "gene": "UniProtKB:O95786",
  "term_label": "cytoplasm",
  "term_id": "GO:0005737"
}